{
  "gene": "UniProtKB:Q9UK45",
  "gene_name": "U6 snRNA-associated Sm-like protein LSm7",
  "gene_symbol": "LSM7",
  "term_label": "RNA binding",
  "term_id": "GO:0003723"
}